{
  "term_label": "phospholipid translocation",
  "gene_symbol": "ATP10D",
  "gene": "UniProtKB:Q9P241",
  "term_id": "GO:0045332",
  "gene_name": "Phospholipid-transporting ATPase VD"
}